{
  "gene_symbol": "XRCC3",
  "gene_name": "DNA repair protein XRCC3",
  "gene": "UniProtKB:O43542",
  "term_id": "GO:0033065",
  "term_label": "Rad51C-XRCC3 complex"
}